{
  "gene": "UniProtKB:P32302",
  "gene_name": "C-X-C chemokine receptor type 5",
  "term_label": "external side of plasma membrane",
  "gene_symbol": "CXCR5",
  "term_id": "GO:0009897"
}